{
  "gene": "UniProtKB:Q9BW60",
  "gene_name": "Elongation of very long chain fatty acids protein 1",
  "term_label": "fatty acid elongation, polyunsaturated fatty acid",
  "gene_symbol": "ELOVL1",
  "term_id": "GO:0034626"
}